post-embryonic caudal fin morphogenesis [GO:0035133] (biological process) Sources: GOC:dgh Relationships: is_a post-embryonic medial fin morphogenesis [GO:0035132]; is a type of GO:0035143 Definition: The process, occurring after embryonic development, by which the anatomical structures of the caudal fin are generated and organized. The caudal fin is an unpaired medial fin mounted at the caudal end of the fish and is the main fin used for propulsion.